{
  "term_label": "Unknown molecular function",
  "gene_name": "Integrator complex subunit 8",
  "gene_symbol": "INTS8",
  "gene": "UniProtKB:Q75QN2",
  "term_id": "UNKNOWN:0001"
}